{
  "term_label": "receptor guanylyl cyclase signaling pathway",
  "gene_name": "Atrial natriuretic peptide receptor 2",
  "term_id": "GO:0007168",
  "gene": "UniProtKB:P20594",
  "gene_symbol": "NPR2"
}